{
  "term_id": "GO:0005201",
  "gene_name": "Protein eyes shut homolog",
  "gene": "UniProtKB:Q5T1H1",
  "gene_symbol": "EYS",
  "term_label": "extracellular matrix structural constituent"
}